{
  "gene_symbol": "SERGEF",
  "gene": "UniProtKB:Q9UGK8",
  "term_id": "GO:0005634",
  "term_label": "nucleus",
  "gene_name": "Secretion-regulating guanine nucleotide exchange factor"
}